{
  "gene": "UniProtKB:Q8IWA0",
  "term_id": "GO:2000234",
  "gene_symbol": "WDR75",
  "term_label": "positive regulation of rRNA processing",
  "gene_name": "WD repeat-containing protein 75"
}